{
  "gene": "UniProtKB:A6NER3",
  "gene_symbol": "GAGE12J",
  "term_label": "Unknown molecular function",
  "gene_name": "G antigen 12J",
  "term_id": "UNKNOWN:0001"
}